{
  "gene_symbol": "PRM2",
  "gene": "UniProtKB:P04554",
  "gene_name": "Protamine-2",
  "term_id": "GO:0005634",
  "term_label": "nucleus"
}